positive regulation of palmitic acid catabolic process [GO:0106395] (biological process) Definition: Any process that activates or increases the frequency, rate or extent of a palmitic acid catabolic process. Relationships: is a type of positive regulation of fatty acid metabolic process [GO:0045923]; is a type of positive regulation of lipid catabolic process [GO:0050996]; is a type of GO:0106393; positively regulates palmitic acid catabolic process [GO:1900534] References: PMID:14677856